{
  "gene_symbol": "ZNF566",
  "term_label": "RNA polymerase II transcription regulatory region sequence-specific DNA binding",
  "gene": "UniProtKB:Q969W8",
  "gene_name": "Zinc finger protein 566",
  "term_id": "GO:0000977"
}